{
  "gene_symbol": "SPINT3",
  "gene": "UniProtKB:P49223",
  "gene_name": "Kunitz-type protease inhibitor 3",
  "term_label": "Unknown molecular function",
  "term_id": "UNKNOWN:0001"
}